{
  "term_id": "GO:0048188",
  "gene_name": "WD repeat-containing protein 5B",
  "gene_symbol": "WDR5B",
  "term_label": "Set1C/COMPASS complex",
  "gene": "UniProtKB:Q86VZ2"
}